{
  "term_id": "UNKNOWN:0001",
  "gene_symbol": "TMEM14B",
  "gene": "UniProtKB:Q9NUH8",
  "gene_name": "Transmembrane protein 14B",
  "term_label": "Unknown molecular function"
}